{
  "term_label": "cysteine-type deubiquitinase activity",
  "gene": "UniProtKB:Q9NVE5",
  "term_id": "GO:0004843",
  "gene_symbol": "USP40",
  "gene_name": "Ubiquitin carboxyl-terminal hydrolase 40"
}